{
  "gene_name": "Fractalkine",
  "gene_symbol": "CX3CL1",
  "gene": "UniProtKB:P78423",
  "term_id": "GO:0048020",
  "term_label": "CCR chemokine receptor binding"
}